{
  "term_id": "GO:0005737",
  "gene": "UniProtKB:A4D1U4",
  "gene_name": "DENN domain-containing protein 11",
  "term_label": "cytoplasm",
  "gene_symbol": "DENND11"
}